{
  "gene_symbol": "PNLIPRP3",
  "term_label": "fatty acid biosynthetic process",
  "gene": "UniProtKB:Q17RR3",
  "gene_name": "Pancreatic lipase-related protein 3",
  "term_id": "GO:0006633"
}